{
  "gene_name": "Metallothionein-1G",
  "gene": "UniProtKB:P13640",
  "term_label": "intracellular zinc ion homeostasis",
  "gene_symbol": "MT1G",
  "term_id": "GO:0006882"
}